response to caffeine [GO:0031000] (biological process) Definition: Any process that results in a change in state or activity of a cell or an organism (in terms of movement, secretion, enzyme production, gene expression, etc.) as a result of a caffeine stimulus. Caffeine is an alkaloid found in numerous plant species, where it acts as a natural pesticide that paralyzes and kills certain insects feeding upon them. Sources: GOC:ef, GOC:mah Subtypes: cellular response to caffeine [GO:0071313] Relationships: is a type of response to purine-containing compound [GO:0014074]; is a type of GO:0043279